follicular dendritic cell differentiation [GO:0002268] (biological process) Definition: The process in which a relatively unspecialized precursor cell acquires the specialized features of a follicular dendritic cell. Sources: GOC:add, ISBN:0781735149 Relationships: is a type of follicular dendritic cell activation [GO:0002266]; is a type of cell differentiation [GO:0030154]